{
  "gene_name": "Aurora kinase C",
  "term_label": "regulation of cytokinesis",
  "gene_symbol": "AURKC",
  "term_id": "GO:0032465",
  "gene": "UniProtKB:Q9UQB9"
}